{
  "gene": "UniProtKB:P04632",
  "gene_symbol": "CAPNS1",
  "term_label": "Unknown biological process",
  "term_id": "UNKNOWN:0002",
  "gene_name": "Calpain small subunit 1"
}